{
  "gene": "UniProtKB:Q1EHB4",
  "gene_symbol": "SLC5A12",
  "term_label": "Unknown cellular component",
  "gene_name": "Sodium-coupled monocarboxylate transporter 2",
  "term_id": "UNKNOWN:0003"
}